{
  "gene_symbol": "HMGB1",
  "gene": "UniProtKB:P09429",
  "term_id": "UNKNOWN:0001",
  "term_label": "Unknown molecular function",
  "gene_name": "High mobility group protein B1"
}